lipid-linked peptidoglycan transport [GO:0015836] (biological process) Also known as: lipid-linked murein transport Relationships: is a type of GO:0015835 Sources: GOC:mah Definition: The directed movement of lipid-linked peptidoglycans into, out of or within a cell, or between cells, by means of some agent such as a transporter or pore.